{
  "term_id": "GO:0005634",
  "gene_symbol": "AGAP3",
  "gene": "UniProtKB:Q96P47",
  "term_label": "nucleus",
  "gene_name": "Arf-GAP with GTPase, ANK repeat and PH domain-containing protein 3"
}